extracellular microvesicle biogenesis [GO:0140113] (BP) Definition: The assembly and secretion of a set of components to form an extracellular microvesicule, a membrane-bounded vesicle that ranges in size 100 nm to 1 micron in size) and exits the cell by budding. References: PMID:28736435 Relationships: is a type of extracellular vesicle biogenesis [GO:0140112] Also known as: extracellular microvesicle assembly